{
  "term_id": "GO:0042450",
  "gene_symbol": "OTC",
  "gene_name": "Ornithine transcarbamylase, mitochondrial",
  "term_label": "L-arginine biosynthetic process via ornithine",
  "gene": "UniProtKB:P00480"
}